{
  "term_id": "GO:0005667",
  "gene_name": "Nuclear factor of activated T-cells 5",
  "term_label": "transcription regulator complex",
  "gene_symbol": "NFAT5",
  "gene": "UniProtKB:O94916"
}